cell development [GO:0048468] (biological process) Relationships: is a type of GO:0048856; is a type of cellular developmental process [GO:0048869]; BFO_0000050 cell differentiation [GO:0030154] Also known as: terminal differentiation Regulation: RO_0002213 by positive regulation of cell development [GO:0010720]; negatively regulated by GO:0010721; regulated by regulation of cell development [GO:0060284] Subtypes: chlamydospore formation [GO:0001410], chondrocyte development [GO:0002063], GO:0002064, osteoblast development [GO:0002076], corneocyte development [GO:0003335], pole cell development [GO:0007277], GO:0007281, oenocyte development [GO:0007438], guard cell development [GO:0010441], neuroblast development [GO:0014019], GO:0014031, glial cell development [GO:0021782], hemopoiesis [GO:0030097], eosinophil differentiation [GO:0030222], ascospore formation [GO:0030437], myoblast development [GO:0048627], neuron development [GO:0048666], stem cell development [GO:0048864], muscle cell development [GO:0055001], cardiac cell development [GO:0055006], GO:0060035, corticotropin hormone secreting cell development [GO:0060131], prolactin secreting cell development [GO:0060132], somatotropin secreting cell development [GO:0060133], GO:0060719, establishment of blood-brain barrier [GO:0060856], conidium development [GO:0061794], GO:0070285, metula development [GO:0070789], GO:0070790, GO:0070792, GO:0072140, renal interstitial fibroblast development [GO:0072141], juxtaglomerulus cell development [GO:0072142], GO:0072143, proximal convoluted tubule segment 1 cell development [GO:0072145], spore encystment [GO:0075214], root hair cell development [GO:0080147], sepal giant cell development [GO:0090393], leaf pavement cell development [GO:0090436], GO:0098751, establishment of blood-retinal barrier [GO:1990963] Sources: GOC:go_curators Definition: The cellular developmental process in which a specific cell progresses from an immature to a mature state. Cell development start once cell commitment has taken place.